{
  "gene_symbol": "SAGE1",
  "gene_name": "Sarcoma antigen 1",
  "gene": "UniProtKB:Q9NXZ1",
  "term_id": "GO:0030674",
  "term_label": "protein-macromolecule adaptor activity"
}